{
  "gene_symbol": "PSEN2",
  "gene": "UniProtKB:P49810",
  "term_id": "GO:0007219",
  "term_label": "Notch signaling pathway",
  "gene_name": "Presenilin-2"
}